{
  "gene": "UniProtKB:Q9H898",
  "gene_name": "Zinc finger matrin-type protein 4",
  "term_label": "Unknown cellular component",
  "term_id": "UNKNOWN:0003",
  "gene_symbol": "ZMAT4"
}